{
  "gene_symbol": "SLC9A7",
  "term_label": "potassium ion transmembrane transport",
  "gene": "UniProtKB:Q96T83",
  "gene_name": "Sodium_hydrogen exchanger 7",
  "term_id": "GO:0071805"
}